{
  "gene_name": "Cytochrome b-c1 complex subunit 8",
  "gene": "UniProtKB:O14949",
  "term_id": "GO:0006122",
  "term_label": "mitochondrial electron transport, ubiquinol to cytochrome c",
  "gene_symbol": "UQCRQ"
}